positive regulation of establishment of bipolar cell polarity [GO:0061173] (biological process) Relationships: is a type of GO:0048522; is_a GO:0061172; positively regulates establishment of bipolar cell polarity [GO:0061171] Sources: GOC:dph, GOC:vw Definition: Any process that increases the rate, frequency or extent of the establishment of bipolar cell polarity. Subtypes: positive regulation of establishment of bipolar cell polarity regulating cell shape [GO:0061161]